ciliary vesicle [GO:0097721] (CC) Definition: A Golgi-derived vesicle to which the ciliary basal body docks via its transitional fibers. Its membrane is compositionally distinct from Golgi membranes, and will become the ciliary membrane once the ciliary vesicle is fused to the plasma membrane. The ciliary vesicle is thought to be formed by multiple smaller vesicles that attach to the transitional fibers and then fuse to form a larger vesicle. References: PMID:13978319, PMID:25686250 Sources: GOC:cilia Also known as: primary ciliary vesicle, CV Relationships: is a type of cytoplasmic vesicle [GO:0031410]